{
  "gene": "UniProtKB:A0A0G2JS06",
  "gene_symbol": "IGLV5-39",
  "gene_name": "Immunoglobulin lambda variable 5-39",
  "term_id": "UNKNOWN:0001",
  "term_label": "Unknown molecular function"
}